{
  "gene_symbol": "HLA-DOA",
  "term_label": "positive regulation of immune response",
  "gene": "UniProtKB:P06340",
  "gene_name": "HLA class II histocompatibility antigen, DO alpha chain",
  "term_id": "GO:0050778"
}